{
  "gene_symbol": "TRIM50",
  "term_label": "ubiquitin protein ligase activity",
  "term_id": "GO:0061630",
  "gene_name": "E3 ubiquitin-protein ligase TRIM50",
  "gene": "UniProtKB:Q86XT4"
}